{
  "term_id": "GO:0005667",
  "gene_symbol": "TEAD3",
  "term_label": "transcription regulator complex",
  "gene": "UniProtKB:Q99594",
  "gene_name": "Transcriptional enhancer factor TEF-5"
}